{
  "term_id": "GO:1901224",
  "gene_symbol": "SASH1",
  "gene": "UniProtKB:O94885",
  "gene_name": "SAM and SH3 domain-containing protein 1",
  "term_label": "positive regulation of non-canonical NF-kappaB signal transduction"
}